L-glutamine transmembrane transporter activity [GO:0015186] (molecular function) Definition: Enables the transfer of L-glutamine from one side of a membrane to the other. L-glutamine is 2-amino-4-carbamoylbutanoic acid. Also known as: asparagine/glutamine permease activity Subtypes: high-affinity glutamine transmembrane transporter activity [GO:0015330], ATPase-coupled L-glutamine transmembrane transporter activity [GO:0015599], GO:0140830, L-glutamine:sodium symporter activity [GO:0140902] Relationships: is a type of neutral L-amino acid transmembrane transporter activity [GO:0015175]; is a type of L-amino acid transmembrane transporter activity [GO:0015179]; is part of GO:0006868 Sources: GOC:ai, GOC:mtg_transport, ISBN:0815340729